{
  "term_label": "dynein light intermediate chain binding",
  "gene_symbol": "HOOK1",
  "gene": "UniProtKB:Q9UJC3",
  "term_id": "GO:0051959",
  "gene_name": "Protein Hook homolog 1"
}